{
  "gene": "UniProtKB:P19419",
  "gene_name": "ETS domain-containing protein Elk-1",
  "term_label": "cell differentiation",
  "term_id": "GO:0030154",
  "gene_symbol": "ELK1"
}